positive regulation of inflammasome-mediated signaling pathway [GO:0141087] (biological process) Definition: Any process that activates or increases the frequency, rate or extent of an inflammasome-mediated signaling pathway. References: PMID:33467177 Also known as: positive regulation of inflammasome-mediated signal transduction Relationships: is a type of GO:0062208; is a type of GO:0141085; is a type of positive regulation of intracellular signal transduction [GO:1902533]; positively regulates GO:0141084